1,1,1-trichloro-2,2-bis-(4-chlorophenyl)ethane metabolic process [GO:0018977] (biological process) Also known as: 1,1,1-trichloro-2,2-bis-(4-chlorophenyl)ethane metabolism, DDT metabolic process, DDT metabolism Relationships: is a type of insecticide metabolic process [GO:0017143]; is_a halogenated hydrocarbon metabolic process [GO:0042197]; is a type of GO:0042537 Sources: GOC:jl Definition: The chemical reactions and pathways involving 1,1,1-trichloro-2,2-bis-(4-chlorophenyl)ethane (DDT), a chlorinated broad spectrum contact insecticide. Subtypes: anaerobic 1,1,1-trichloro-2,2-bis-(4-chlorophenyl)ethane metabolic process [GO:0018978], 1,1,1-trichloro-2,2-bis-(4-chlorophenyl)ethane catabolic process [GO:0042188]